{
  "gene_name": "Lysine-specific demethylase 4C",
  "gene_symbol": "KDM4C",
  "term_id": "GO:0032454",
  "gene": "UniProtKB:Q9H3R0",
  "term_label": "histone H3K9 demethylase activity"
}